{
  "term_id": "UNKNOWN:0001",
  "term_label": "Unknown molecular function",
  "gene_name": "Lipocalin_cytosolic fatty-acid binding domain-containing protein",
  "gene_symbol": "LOC102723971",
  "gene": "UniProtKB:A0A1B0GUV8"
}